{
  "term_label": "RNA binding",
  "gene": "UniProtKB:A6NGQ2",
  "gene_name": "Oocyte-expressed protein homolog",
  "term_id": "GO:0003723",
  "gene_symbol": "OOEP"
}